{
  "term_label": "Unknown biological process",
  "term_id": "UNKNOWN:0002",
  "gene": "UniProtKB:P63128",
  "gene_name": "Endogenous retrovirus group K member 9 Pol protein",
  "gene_symbol": "ERVK-9"
}